{
  "term_id": "GO:0031647",
  "gene": "UniProtKB:Q9UHP3",
  "gene_name": "Ubiquitin carboxyl-terminal hydrolase 25",
  "gene_symbol": "USP25",
  "term_label": "regulation of protein stability"
}